{
  "gene": "UniProtKB:P98170",
  "gene_symbol": "XIAP",
  "term_label": "ubiquitin protein ligase activity",
  "gene_name": "E3 ubiquitin-protein ligase XIAP",
  "term_id": "GO:0061630"
}